{
  "term_id": "GO:0090051",
  "gene_symbol": "MMRN1",
  "gene_name": "Multimerin-1",
  "gene": "UniProtKB:Q13201",
  "term_label": "negative regulation of cell migration involved in sprouting angiogenesis"
}